{
  "term_id": "GO:0055088",
  "gene_name": "Patatin-like phospholipase domain-containing protein 4",
  "term_label": "lipid homeostasis",
  "gene": "UniProtKB:P41247",
  "gene_symbol": "PNPLA4"
}